{
  "term_label": "cytoplasm",
  "gene": "UniProtKB:P78362",
  "gene_name": "SRSF protein kinase 2",
  "term_id": "GO:0005737",
  "gene_symbol": "SRPK2"
}